peptidoglycan N-acetylglucosaminidase activity [GO:0061784] (molecular function) Definition: Catalysis of the hydrolysis of (1->4)-beta linkages of N-acetyl-D-glucosamine (GlcNAc) from peptidoglycan. References: PMID:22748813 Sources: GOC:dph, GOC:jh Relationships: is a type of GO:0015929; is a type of GO:0061783